oxidoreductase activity, acting on the CH-NH group of donors, disulfide as acceptor [GO:0016648] (molecular function) Sources: GOC:jl Subtypes: pyrimidodiazepine synthase activity [GO:0004734] Definition: Catalysis of an oxidation-reduction (redox) reaction in which a CH-NH group acts as a hydrogen or electron donor and reduces disulfide. Relationships: is a type of GO:0016645 Also known as: oxidoreductase activity, acting on the CH-NH group of donors, disulphide as acceptor